{
  "gene_symbol": "ZNF747",
  "term_id": "GO:0000122",
  "gene_name": "Zinc finger protein 747",
  "gene": "UniProtKB:Q9BV97",
  "term_label": "negative regulation of transcription by RNA polymerase II"
}